{
  "gene_symbol": "UBQLN2",
  "term_label": "ubiquitin-dependent protein catabolic process",
  "gene": "UniProtKB:Q9UHD9",
  "term_id": "GO:0006511",
  "gene_name": "Ubiquilin-2"
}